{
  "gene_name": "Alpha-crystallin A chain",
  "gene": "UniProtKB:P02489",
  "gene_symbol": "CRYAA",
  "term_id": "GO:0051082",
  "term_label": "unfolded protein binding"
}